{
  "gene_name": "Aspartate aminotransferase, mitochondrial",
  "gene": "UniProtKB:P00505",
  "gene_symbol": "GOT2",
  "term_id": "GO:0005739",
  "term_label": "mitochondrion"
}